cadinene biosynthetic process [GO:1901928] (BP) References: PMID:22867794 Sources: GOC:TermGenie Definition: The chemical reactions and pathways resulting in the formation of cadinene. Also known as: cadinene anabolism, cadinene biosynthesis, cadinene formation, cadinene synthesis Relationships: is_a sesquiterpene biosynthetic process [GO:0051762]